{
  "gene": "UniProtKB:Q9ULV0",
  "term_id": "GO:0000146",
  "gene_symbol": "MYO5B",
  "gene_name": "Unconventional myosin-Vb",
  "term_label": "microfilament motor activity"
}